formaldehyde assimilation [GO:0019649] (biological process) Subtypes: formaldehyde assimilation via ribulose monophosphate cycle [GO:0019647], formaldehyde assimilation via xylulose monophosphate cycle [GO:0019648] Definition: The pathways in which formaldehyde is processed and used as a carbon source for the cell. Sources: GOC:ai Relationships: is a type of formaldehyde metabolic process [GO:0046292]